type B pancreatic cell development [GO:0003323] (biological process) Also known as: pancreatic B cell development, pancreatic beta cell development Regulation: regulated by regulation of type B pancreatic cell development [GO:2000074]; negatively regulated by negative regulation of type B pancreatic cell development [GO:2000077]; positively regulated by positive regulation of type B pancreatic cell development [GO:2000078] Definition: The process whose specific outcome is the progression of a type B pancreatic cell over time, from its formation to the mature structure. A type B pancreatic cell is a cell located towards center of the islets of Langerhans that secretes insulin. Sources: CL:0000169, GOC:dph Relationships: is a type of epithelial cell development [GO:0002064]; is part of GO:0003309